{
  "gene_symbol": "HNRNPC",
  "gene_name": "Heterogeneous nuclear ribonucleoproteins C1_C2",
  "term_label": "nucleus",
  "term_id": "GO:0005634",
  "gene": "UniProtKB:P07910"
}